{
  "gene": "UniProtKB:Q5VU57",
  "gene_name": "Cytosolic carboxypeptidase 6",
  "gene_symbol": "AGBL4",
  "term_label": "tubulin binding",
  "term_id": "GO:0015631"
}